{
  "term_label": "cell surface receptor protein tyrosine kinase signaling pathway",
  "gene_symbol": "PDGFRA",
  "gene": "UniProtKB:P16234",
  "term_id": "GO:0007169",
  "gene_name": "Platelet-derived growth factor receptor alpha"
}